{
  "gene": "UniProtKB:P49959",
  "gene_name": "Double-strand break repair protein MRE11",
  "term_label": "mitotic intra-S DNA damage checkpoint signaling",
  "gene_symbol": "MRE11",
  "term_id": "GO:0031573"
}